{
  "gene_name": "Protein SON",
  "gene_symbol": "SON",
  "term_label": "RNA binding",
  "term_id": "GO:0003723",
  "gene": "UniProtKB:P18583"
}